{
  "gene_symbol": "ZNF486",
  "term_label": "regulation of DNA-templated transcription",
  "gene": "UniProtKB:Q96H40",
  "gene_name": "Zinc finger protein 486",
  "term_id": "GO:0006355"
}